FAD-dependent urate hydroxylase activity [GO:0102099] (molecular function) Relationships: is_a oxidoreductase activity, acting on paired donors, with incorporation or reduction of molecular oxygen, NAD(P)H as one donor, and incorporation of one atom of oxygen [GO:0016709] Definition: Catalysis of the reaction: 7,9-dihydro-1H-purine-2,6,8(3H)-trione + NADH + H+ + O2 = 5-hydroxyisouric acid + NAD + H2O. Sources: EC:1.14.13.113, GOC:pz